regulation of cardiac muscle contraction by regulation of the release of sequestered calcium ion [GO:0010881] (biological process) Definition: Any process that modulates the frequency, rate or extent of cardiac muscle contraction via the regulation of the release of sequestered calcium ion by sarcoplasmic reticulum into cytosol. The sarcoplasmic reticulum is the endoplasmic reticulum of striated muscle, specialised for the sequestration of calcium ions that are released upon receipt of a signal relayed by the T tubules from the neuromuscular junction. Sources: GOC:BHF, GOC:dph, GOC:tb Relationships: is a type of GO:0010880; is a type of GO:0010882